{
  "gene_name": "Myotubularin-related protein 2",
  "gene_symbol": "MTMR2",
  "gene": "UniProtKB:Q13614",
  "term_id": "GO:0016020",
  "term_label": "membrane"
}